{
  "term_id": "GO:0006508",
  "term_label": "proteolysis",
  "gene_name": "Calpain-12",
  "gene": "UniProtKB:Q6ZSI9",
  "gene_symbol": "CAPN12"
}